{
  "term_id": "GO:0061824",
  "gene": "UniProtKB:Q5JSH3",
  "term_label": "cytosolic ciliogenesis",
  "gene_name": "WD repeat-containing protein 44",
  "gene_symbol": "WDR44"
}